{
  "term_id": "GO:0072675",
  "gene_name": "T-cell leukemia translocation-altered gene protein",
  "gene_symbol": "TCTA",
  "term_label": "osteoclast fusion",
  "gene": "UniProtKB:P57738"
}